{
  "gene_symbol": "MSL2",
  "term_label": "MSL complex",
  "gene_name": "E3 ubiquitin-protein ligase MSL2",
  "term_id": "GO:0072487",
  "gene": "UniProtKB:Q9HCI7"
}